{
  "gene_name": "Tumor necrosis factor ligand superfamily member 8",
  "term_label": "Unknown cellular component",
  "gene_symbol": "TNFSF8",
  "gene": "UniProtKB:P32971",
  "term_id": "UNKNOWN:0003"
}